{
  "gene_name": "Mothers against decapentaplegic homolog 2",
  "gene_symbol": "SMAD2",
  "term_label": "activin receptor signaling pathway",
  "gene": "UniProtKB:Q15796",
  "term_id": "GO:0032924"
}